{
  "term_label": "negative regulation of Wnt signaling pathway",
  "gene": "UniProtKB:Q6DKJ4",
  "term_id": "GO:0030178",
  "gene_symbol": "NXN",
  "gene_name": "Nucleoredoxin"
}